{
  "gene": "UniProtKB:O60784",
  "term_label": "signal transduction",
  "gene_name": "Target of Myb1 membrane trafficking protein",
  "term_id": "GO:0007165",
  "gene_symbol": "TOM1"
}